{
  "gene_name": "LYR motif-containing protein 2",
  "gene": "UniProtKB:Q9NU23",
  "term_label": "Unknown biological process",
  "gene_symbol": "LYRM2",
  "term_id": "UNKNOWN:0002"
}